{
  "gene_name": "Keratin, type I cytoskeletal 14",
  "term_id": "GO:0030216",
  "gene": "UniProtKB:P02533",
  "term_label": "keratinocyte differentiation",
  "gene_symbol": "KRT14"
}